{
  "gene_name": "Protein PRR14L",
  "gene": "UniProtKB:Q5THK1",
  "gene_symbol": "PRR14L",
  "term_label": "Unknown cellular component",
  "term_id": "UNKNOWN:0003"
}